{
  "gene": "UniProtKB:Q9NTI2",
  "gene_name": "Phospholipid-transporting ATPase IB",
  "term_id": "GO:0005886",
  "term_label": "plasma membrane",
  "gene_symbol": "ATP8A2"
}